{
  "gene_symbol": "SPATA32",
  "gene": "UniProtKB:Q96LK8",
  "term_id": "GO:0003779",
  "term_label": "actin binding",
  "gene_name": "Spermatogenesis-associated protein 32"
}